{
  "gene_name": "Pre-mRNA-splicing factor ATP-dependent RNA helicase PRP16",
  "gene": "UniProtKB:Q92620",
  "term_label": "mRNA splicing, via spliceosome",
  "gene_symbol": "DHX38",
  "term_id": "GO:0000398"
}